lysine biosynthetic process via alpha-aminoadipate and N2-acetyl-alpha-aminoadipate [GO:0051976] (BP) Definition: The chemical reactions and pathways resulting in the formation of lysine via the intermediates alpha-aminoadipic acid and N2-acetyl-alpha-aminoadipate. This pathway of prokaryotic lysine biosynthesis via alpha-aminoadipate was discovered in the hyper-thermophilic Gram-negative eubacterium Thermus thermophilus. The pathway proceeds as follows: alpha-ketoglutarate is converted to homocitrate, which is metabolized to 3-carboxyhex-2-enedioate and then homoisocitrate. This is then decarboxylated to form alpha-ketoadipate, which is then converted to alpha-aminoadipate. This undergoes acetylation, to form N2-acetyl-alpha-aminoadipate, and is then phosphorylated to give N2-acetyl-alpha-aminoadipyl-delta-phosphate. This is converted to N2-acetyl-alpha-aminoadipate semialdehyde, which is then converted to N2-acetyl-L-lysine. A final deacetylation reaction produces L-lysine. Sources: MetaCyc:PWY-3081 Also known as: lysine biosynthesis via aminoadipic acid and N2-acetyl-alpha-aminoadipate, lysine biosynthetic process via aminoadipic acid and N2-acetyl-alpha-aminoadipate Relationships: is a type of lysine biosynthetic process via aminoadipic acid [GO:0019878]